{
  "term_label": "cytoplasm",
  "gene_name": "Ornithine aminotransferase, mitochondrial",
  "gene_symbol": "OAT",
  "term_id": "GO:0005737",
  "gene": "UniProtKB:P04181"
}